{
  "term_id": "UNKNOWN:0001",
  "gene_name": "Golgi-associated RAB2 interactor protein 1A",
  "gene_symbol": "GARIN1A",
  "gene": "UniProtKB:Q6NXP2",
  "term_label": "Unknown molecular function"
}